negative regulation of cellular response to nitrogen starvation [GO:0010516] (biological process) Definition: Any process that stops, prevents, or reduces the frequency, rate or extent of a cellular response to nitrogen starvation. Sources: GOC:dph, GOC:tb Relationships: is a type of negative regulation of response to nutrient levels [GO:0032108]; is a type of negative regulation of cellular process [GO:0048523]; is a type of regulation of cellular response to stress [GO:0080135]; negatively regulates cellular response to nitrogen starvation [GO:0006995]